molybdate ion transport [GO:0015689] (biological process) Subtypes: GO:0090414 Relationships: is_a GO:0015698 Definition: The directed movement of molybdate (MoO4 2-) ions into, out of or within a cell, or between cells, by means of some agent such as a transporter or pore. Molybdate is the bivalent anion derived from molybdic acid. Sources: GOC:ai